response to papulacandin B [GO:0072730] (BP) Subtypes: cellular response to papulacandin B [GO:0072731] Definition: Any process that results in a change in state or activity of a cell or an organism (in terms of movement, secretion, enzyme production, gene expression, etc.) as a result of a papulacandin B stimulus. Relationships: is_a GO:0033993; is a type of response to oxygen-containing compound [GO:1901700] Sources: GOC:mah